hydrogen peroxide channel activity [GO:0140070] (molecular function) Definition: Enables the energy-independent facilitated diffusion of hydrogen peroxide through a transmembrane aqueous pore or channel. References: PMID:23541115, PMID:27256569 Also known as: hydrogen peroxide transmembrane transporter activity Relationships: is a type of GO:0015267; is part of hydrogen peroxide transmembrane transport [GO:0080170]